thiosulfate binding [GO:0036173] (molecular function) References: PMID:2188959 Sources: GOC:db Relationships: is_a anion binding [GO:0043168]; is a type of sulfur compound binding [GO:1901681] Definition: Binding to a thiosulfate, a sulfur oxide that has formula O3S2.